SUMO polymer binding [GO:0032184] (molecular function) Relationships: is a type of SUMO binding [GO:0032183] Definition: Binding to a polymer of the small ubiquitin-like protein SUMO. Also known as: Smt3 polymer binding Sources: GOC:mah